regulation of collateral sprouting of intact axon in response to injury [GO:0048683] (biological process) Definition: Any process that modulates the frequency, rate or extent of collateral sprouting of an intact axon as a result of injury to an axon. Relationships: is a type of GO:0048670; is a type of regulation of axon regeneration [GO:0048679]; regulates GO:0048673 Sources: GOC:dgh, GOC:dph, GOC:jid, GOC:lm Subtypes: GO:0048684, negative regulation of collateral sprouting of intact axon in response to injury [GO:0048685]